mercury ion transmembrane transporter activity [GO:0015097] (molecular function) Definition: Enables the transfer of mercury (Hg2+) ions from one side of a membrane to the other. Sources: GOC:ai Relationships: is a type of GO:0046915; is part of mercury ion transport [GO:0015694]